{
  "gene_name": "Interferon-induced transmembrane protein 3",
  "term_id": "GO:0035455",
  "gene_symbol": "IFITM3",
  "gene": "UniProtKB:Q01628",
  "term_label": "response to interferon-alpha"
}